{
  "gene_name": "Protein lifeguard 4",
  "term_label": "membrane",
  "term_id": "GO:0016020",
  "gene_symbol": "TMBIM4",
  "gene": "UniProtKB:Q9HC24"
}